S-methyltransferase activity [GO:0008172] (molecular function) Sources: GOC:ai Definition: Catalysis of the transfer of a methyl group to the sulfur atom of an acceptor molecule. Subtypes: 5-methyltetrahydropteroyltriglutamate-homocysteine S-methyltransferase activity [GO:0003871], GO:0003908, GO:0004790, GO:0008119, methionine synthase activity [GO:0008705], S-adenosylmethionine-homocysteine S-methyltransferase activity [GO:0008898], GO:0018708, tetrahydromethanopterin S-methyltransferase activity [GO:0030269], thetin-homocysteine S-methyltransferase activity [GO:0047149], betaine-homocysteine S-methyltransferase activity [GO:0047150], GO:0061627, protein-cysteine methyltransferase activity [GO:0106363] Relationships: is a type of methyltransferase activity [GO:0008168]